{
  "term_label": "actin cytoskeleton",
  "term_id": "GO:0015629",
  "gene_symbol": "AVIL",
  "gene_name": "Advillin",
  "gene": "UniProtKB:O75366"
}